L-serine-glyoxylate transaminase activity [GO:0050281] (molecular function) Also known as: serine--glyoxylate aminotransferase activity, L-serine:glyoxylate aminotransferase activity, SGAT activity Relationships: is a type of GO:0008483 Sources: EC:2.6.1.45 Definition: Catalysis of the reaction: L-serine + glyoxylate = 3-hydroxypyruvate + glycine.